pons formation [GO:0021584] (biological process) Definition: The process that gives rise to the pons. This process pertains to the initial formation of a structure from unspecified parts. The pons lies above the medulla and next to the cerebellum. The pons conveys information about movement from the cerebral hemisphere to the cerebellum. Relationships: is a type of anatomical structure formation involved in morphogenesis [GO:0048646]; is part of hindbrain formation [GO:0021576]; is part of pons morphogenesis [GO:0021583] Sources: GOC:cls, GOC:dgh, GOC:dph, GOC:jid, GO_REF:0000021